adenosyl-fluoride synthase activity [GO:0033846] (molecular function) Sources: EC:2.5.1.63 Also known as: S-adenosyl-L-methionine:fluoride adenosyltransferase activity, fluorinase activity Definition: Catalysis of the reaction: S-adenosyl-L-methionine + fluoride = 5'-deoxy-5'-fluoroadenosine + L-methionine. Relationships: is_a transferase activity, transferring alkyl or aryl (other than methyl) groups [GO:0016765]